{
  "term_id": "UNKNOWN:0002",
  "gene_name": "Transmembrane protein 185A",
  "gene": "UniProtKB:Q8NFB2",
  "term_label": "Unknown biological process",
  "gene_symbol": "TMEM185A"
}